maltoheptaose catabolic process [GO:2001123] (biological process) Also known as: maltoheptaose catabolism Definition: The chemical reactions and pathways resulting in the breakdown of a maltoheptaose. Sources: GOC:mengo_curators Relationships: is a type of GO:0009313; is a type of maltoheptaose metabolic process [GO:2001122]